positive regulation of tumor necrosis factor (ligand) superfamily member 11 production [GO:2000309] (biological process) Also known as: positive regulation of RANKL production, positive regulation of TNFSF11 production Definition: Any process that activates or increases the frequency, rate or extent of tumor necrosis factor (ligand) superfamily member 11 production. Relationships: is a type of GO:1903557; is a type of regulation of tumor necrosis factor (ligand) superfamily member 11 production [GO:2000307]; positively regulates GO:0072535 Sources: GOC:BHF, GOC:mah